EXT1-EXT2 complex [GO:0120504] (cellular component) Definition: A heterodimeric complex capable of glycosyltransferase activity required for the elongation of heparan sulfate chains. In humans, the complex consists of EXT1 and EXT2. In Drosophila, the complex consists of ttv and sotv. References: PMID:14998928, PMID:36402845, PMID:36593275 Sources: GOC:sjm Also known as: EXT1-EXT2 heparan sulfate biosynthesis complex, exostosin complex Relationships: is a type of transferase complex [GO:1990234]